{
  "gene_symbol": "ROBO3",
  "gene_name": "Roundabout homolog 3",
  "gene": "UniProtKB:Q96MS0",
  "term_label": "axon",
  "term_id": "GO:0030424"
}